{
  "gene_name": "BBSome-interacting protein 1",
  "gene_symbol": "BBIP1",
  "term_label": "Unknown molecular function",
  "gene": "UniProtKB:A8MTZ0",
  "term_id": "UNKNOWN:0001"
}